Wnt signaling pathway involved in somitogenesis [GO:0090244] (biological process) Relationships: is a type of Wnt signaling pathway [GO:0016055]; is part of GO:0001756 Definition: The series of molecular signals initiated by binding of Wnt protein to a frizzled family receptor on the surface of the target cell and ending with a change in cell state that contributes to somitogenesis. Sources: GOC:ascb_2009, GOC:dph, GOC:tb Also known as: Wnt receptor signaling pathway involved in somitogenesis, Wnt receptor signalling, Wnt-activated signaling pathway involved in somitogenesis